{
  "gene_symbol": "LINC00299",
  "gene_name": "Putative uncharacterized protein encoded by LINC00299",
  "gene": "UniProtKB:Q6ZSB3",
  "term_label": "Unknown cellular component",
  "term_id": "UNKNOWN:0003"
}